{
  "term_label": "mitotic spindle organization",
  "gene": "UniProtKB:Q9UQB9",
  "gene_name": "Aurora kinase C",
  "gene_symbol": "AURKC",
  "term_id": "GO:0007052"
}